{
  "gene_symbol": "TWNK",
  "gene_name": "Twinkle mtDNA helicase",
  "gene": "UniProtKB:Q96RR1",
  "term_id": "GO:0005739",
  "term_label": "mitochondrion"
}